{
  "term_id": "GO:0038180",
  "gene": "UniProtKB:P34130",
  "gene_name": "Neurotrophin-4",
  "gene_symbol": "NTF4",
  "term_label": "nerve growth factor signaling pathway"
}